{
  "gene": "UniProtKB:P42285",
  "gene_symbol": "MTREX",
  "term_label": "RNA helicase activity",
  "term_id": "GO:0003724",
  "gene_name": "Exosome RNA helicase MTR4"
}